{
  "gene": "UniProtKB:Q7Z4L9",
  "term_label": "Unknown cellular component",
  "term_id": "UNKNOWN:0003",
  "gene_name": "Protein phosphatase 1 regulatory subunit 42",
  "gene_symbol": "PPP1R42"
}